{
  "term_label": "detoxification of copper ion",
  "gene": "UniProtKB:Q93083",
  "gene_name": "Metallothionein-1L",
  "gene_symbol": "MT1L",
  "term_id": "GO:0010273"
}